{
  "gene_name": "RRP15-like protein",
  "gene_symbol": "RRP15",
  "term_id": "GO:0030687",
  "term_label": "preribosome, large subunit precursor",
  "gene": "UniProtKB:Q9Y3B9"
}